{
  "term_id": "GO:0005815",
  "gene_name": "Kinesin-like protein KIFC1",
  "gene_symbol": "KIFC1",
  "gene": "UniProtKB:Q9BW19",
  "term_label": "microtubule organizing center"
}